cerebellar cortex maturation [GO:0021699] (biological process) Relationships: is a type of anatomical structure maturation [GO:0071695]; is part of cerebellum maturation [GO:0021590]; is part of cerebellar cortex development [GO:0021695] Sources: GOC:cls, GOC:dgh, GOC:dph, GOC:jid, GO_REF:0000021 Definition: A developmental process, independent of morphogenetic (shape) change, that is required for the cerebellar cortex to attain its fully functional state. The cerebellar cortex is a thin mantle of gray matter that covers the surface of each cerebral hemisphere. It has a characteristic morphology with convolutions (gyri) and crevices (sulci) that have specific functions. Six layers of nerve cells and the nerve pathways that connect them comprise the cerebellar cortex. Together, these regions are responsible for the processes of conscious thought, perception, emotion and memory as well as advanced motor function.